{
  "gene": "UniProtKB:Q8NDB6",
  "gene_symbol": "FAM156B",
  "gene_name": "Protein FAM156A_FAM156B",
  "term_id": "UNKNOWN:0003",
  "term_label": "Unknown cellular component"
}